{
  "term_label": "ubiquitin protein ligase activity",
  "gene_symbol": "RFPL4AL1",
  "term_id": "GO:0061630",
  "gene_name": "Ret finger protein-like 4A-like protein 1",
  "gene": "UniProtKB:F8VTS6"
}